negative regulation of RNA catabolic process [GO:1902369] (biological process) Also known as: down regulation of RNA breakdown, down regulation of RNA catabolic process, down regulation of RNA catabolism, down regulation of RNA degradation, down-regulation of RNA breakdown, down-regulation of RNA catabolic process, down-regulation of RNA catabolism, down-regulation of RNA degradation, downregulation of RNA breakdown, downregulation of RNA catabolic process, downregulation of RNA catabolism, downregulation of RNA degradation, negative regulation of RNA breakdown, negative regulation of RNA catabolism, negative regulation of RNA degradation, inhibition of RNA breakdown, inhibition of RNA catabolic process, inhibition of RNA catabolism, inhibition of RNA degradation Relationships: is a type of negative regulation of catabolic process [GO:0009895]; is_a GO:0051253; negatively regulates GO:0006401 Definition: Any process that stops, prevents or reduces the frequency, rate or extent of RNA catabolic process. Subtypes: negative regulation of mitochondrial RNA catabolic process [GO:0000961], RNA stabilization [GO:0043489], negative regulation of tRNA catabolic process [GO:1902371], negative regulation of mRNA catabolic process [GO:1902373], negative regulation of miRNA catabolic process [GO:2000626] References: PMID:16640457 Sources: GOC:TermGenie, GOC:bf